{
  "gene_symbol": "MSLN",
  "term_id": "GO:0009986",
  "term_label": "cell surface",
  "gene": "UniProtKB:Q13421",
  "gene_name": "Mesothelin"
}